{
  "gene_symbol": "BOLA3",
  "term_label": "protein maturation",
  "term_id": "GO:0051604",
  "gene": "UniProtKB:Q53S33",
  "gene_name": "BolA-like protein 3"
}